methylthioadenosine nucleosidase activity [GO:0008930] (molecular function) Definition: Catalysis of the reaction: methylthioadenosine + H2O = adenine + 5-methylthio-D-ribose. Sources: EC:3.2.2.16 Relationships: is a type of purine nucleosidase activity [GO:0008477] Also known as: 5'-methylthioadenosine nucleosidase activity, MTA nucleosidase activity, MeSAdo nucleosidase activity, S-methyl-5'-thioadenosine adeninehyrolase activity, methylthioadenosine methylthioribohydrolase activity